3-hydroxyacyl-CoA dehydratase activity [GO:0018812] (molecular function) Definition: Catalysis of the reaction: a 3-hydroxy-fatty acyl-CoA = a (2E)-enoyl-CoA + H2O. Sources: RHEA:33767 Relationships: is a type of GO:0004300 Subtypes: (2E)-enoyl-CoA hydratase activity [GO:0080023], (2E)-butenoyl-CoA hydratase activity [GO:0120092]